{
  "gene_symbol": "PLA2G2D",
  "gene": "UniProtKB:Q9UNK4",
  "gene_name": "Group IID secretory phospholipase A2",
  "term_label": "phospholipid binding",
  "term_id": "GO:0005543"
}